{
  "term_label": "Golgi apparatus",
  "term_id": "GO:0005794",
  "gene": "UniProtKB:Q9UBX8",
  "gene_name": "Beta-1,4-galactosyltransferase 6",
  "gene_symbol": "B4GALT6"
}